polyketide metabolic process [GO:0030638] (biological process) Definition: The chemical reactions and pathways involving polyketides, any of a diverse group of natural products synthesized via linear poly-beta-ketones, which are themselves formed by repetitive head-to-tail addition of acetyl (or substituted acetyl) units indirectly derived from acetate (or a substituted acetate) by a mechanism similar to that for fatty acid biosynthesis but without the intermediate reductive steps. Subtypes: polyketide biosynthetic process [GO:0030639], polyketide catabolic process [GO:0030640], GO:0033067, daunorubicin metabolic process [GO:0044597], doxorubicin metabolic process [GO:0044598] Also known as: polyketide metabolism Sources: GOC:mah, ISBN:0198506732 Relationships: is a type of GO:0019748